{
  "gene_symbol": "TIFA",
  "term_id": "GO:0043123",
  "term_label": "positive regulation of canonical NF-kappaB signal transduction",
  "gene": "UniProtKB:Q96CG3",
  "gene_name": "TRAF-interacting protein with FHA domain-containing protein A"
}